{
  "gene": "UniProtKB:Q00169",
  "gene_name": "Phosphatidylinositol transfer protein alpha isoform",
  "term_id": "UNKNOWN:0002",
  "gene_symbol": "PITPNA",
  "term_label": "Unknown biological process"
}